{
  "term_label": "axon",
  "gene_symbol": "TH",
  "term_id": "GO:0030424",
  "gene": "UniProtKB:P07101",
  "gene_name": "Tyrosine 3-monooxygenase"
}